{
  "gene": "UniProtKB:Q9NZD2",
  "term_id": "GO:1902387",
  "term_label": "ceramide 1-phosphate binding",
  "gene_name": "Glycolipid transfer protein",
  "gene_symbol": "GLTP"
}